{
  "gene_symbol": "SPINK4",
  "gene_name": "Serine protease inhibitor Kazal-type 4",
  "gene": "UniProtKB:O60575",
  "term_id": "UNKNOWN:0003",
  "term_label": "Unknown cellular component"
}